{
  "term_label": "microtubule-based movement",
  "gene_symbol": "DYNLT3",
  "term_id": "GO:0007018",
  "gene": "UniProtKB:P51808",
  "gene_name": "Dynein light chain Tctex-type 3"
}